{
  "gene_symbol": "MED8",
  "term_label": "regulation of transcription by RNA polymerase II",
  "term_id": "GO:0006357",
  "gene_name": "Mediator of RNA polymerase II transcription subunit 8",
  "gene": "UniProtKB:Q96G25"
}